{
  "term_id": "GO:0004930",
  "gene_name": "G-protein coupled receptor 176",
  "gene": "UniProtKB:Q14439",
  "gene_symbol": "GPR176",
  "term_label": "G protein-coupled receptor activity"
}